{
  "gene": "UniProtKB:Q96M19",
  "term_label": "Unknown biological process",
  "term_id": "UNKNOWN:0002",
  "gene_name": "Putative transmembrane protein encoded by LINC00477",
  "gene_symbol": "LINC00477"
}